{
  "gene": "UniProtKB:O00194",
  "term_id": "GO:0070382",
  "term_label": "exocytic vesicle",
  "gene_name": "Ras-related protein Rab-27B",
  "gene_symbol": "RAB27B"
}